regulation of host-seeking behavior [GO:0032538] (biological process) Definition: Any process that modulates the frequency, rate or extent of any behavior associated with finding a host organism. Subtypes: GO:0032539, positive regulation of host-seeking behavior [GO:0032540] Relationships: is a type of regulation of behavior [GO:0050795]; regulates host-seeking behavior [GO:0032537] Also known as: regulation of host-seeking behaviour Sources: GOC:mah